{
  "gene_name": "Phospholipid-transporting ATPase IG",
  "term_id": "GO:0005886",
  "gene": "UniProtKB:Q8NB49",
  "term_label": "plasma membrane",
  "gene_symbol": "ATP11C"
}